Mst2 histone acetyltransferase complex [GO:0036410] (cellular component) Definition: A protein complex that can catalyze the acetylation of lysine at position 14 in histone H3, and contains Mst2 as the catalytic subunit. In fission yeast, contains at least Mst2, Nto1, Ptf2, Ptf1 and Eaf6. References: PMID:21289066 Sources: GOC:vw Relationships: is a type of histone H3-K14 acetyltransferase complex [GO:0036409] Also known as: Mst2 H3K14 acetyltransferase complex, Mst2 complex, Mst2 histone H3K14 acetyltransferase complex